{
  "gene_symbol": "NUDT10",
  "gene": "UniProtKB:Q8NFP7",
  "term_label": "diphosphoinositol-polyphosphate diphosphatase activity",
  "term_id": "GO:0008486",
  "gene_name": "Diphosphoinositol polyphosphate phosphohydrolase 3-alpha"
}